phosphatidylinositol alpha-mannosyltransferase activity [GO:0043750] (molecular function) Relationships: is a type of hexosyltransferase activity [GO:0016758] Sources: EC:2.4.1.345 Also known as: GDP mannose-phosphatidyl-myo-inositol alpha-mannosyltransferase activity, GDP mannose:1-phosphatidyl-myo-inositol alpha-D-mannosyltransferase activity, GDP-mannose:1-phosphatidyl-1D-myo-inositol alpha-D-mannosyltransferase activity, GDPmannose:1-phosphatidyl-myo-inositol alpha-D-mannosyltransferase activity, guanosine diphosphomannose-phosphatidyl-inositol alpha-mannosyltransferase activity, phosphatidyl-myo-inositol alpha-mannosyltransferase activity Definition: Catalysis of the transfer of one or more alpha-D-mannose residues from GDP-mannose to positions 2,6 and others in 1-phosphatidyl-myo-inositol.